anti-sigma factor antagonist activity [GO:0043856] (molecular function) References: PMID:15576799 Sources: GOC:jl, GOC:txnOH Relationships: is a type of transcription regulator activity [GO:0140110]; is part of GO:0045893 Also known as: anti-anti-sigma factor activity Definition: The function of binding to an anti-sigma factor and stopping, preventing or reducing the rate of its activity.